positive regulation of extrathymic T cell differentiation [GO:0033090] (biological process) Note: Note that immunologists typically use the word 'development' to refer to cells of B or T cell lineages undergoing the process that GO describes as 'cell differentiation'. Also known as: positive regulation of extrathymic T cell development Relationships: is a type of regulation of extrathymic T cell differentiation [GO:0033082]; is_a positive regulation of T cell differentiation [GO:0045582]; positively regulates extrathymic T cell differentiation [GO:0033078] Sources: GOC:add, GOC:mah Definition: Any process that activates or increases the frequency, rate or extent of extrathymic T cell differentiation.